lymphocyte migration [GO:0072676] (biological process) Relationships: is a type of mononuclear cell migration [GO:0071674] Regulation: regulated by regulation of lymphocyte migration [GO:2000401]; negatively regulated by negative regulation of lymphocyte migration [GO:2000402]; positively regulated by positive regulation of lymphocyte migration [GO:2000403] Subtypes: lymphocyte chemotaxis [GO:0048247], T cell migration [GO:0072678], lymphocyte migration into lymphoid organs [GO:0097021] Sources: CL:0000542, GOC:BHF, GOC:mah Definition: The movement of a lymphocyte within or between different tissues and organs of the body.